prostaglandin biosynthetic process [GO:0001516] (biological process) Relationships: is a type of GO:0006693; is a type of GO:0046457 Subtypes: regulation of fever generation by prostaglandin biosynthetic process [GO:0100008] Regulation: regulated by GO:0031392; RO_0002212 by negative regulation of prostaglandin biosynthetic process [GO:0031393]; positively regulated by GO:0031394 Sources: GOC:ai Also known as: prostaglandin anabolism, prostaglandin biosynthesis, prostaglandin formation, prostaglandin synthesis Definition: The chemical reactions and pathways resulting in the formation of prostaglandins, any of a group of biologically active metabolites which contain a cyclopentane ring.